{
  "term_label": "microtubule binding",
  "gene_symbol": "KIF9",
  "term_id": "GO:0008017",
  "gene": "UniProtKB:Q9HAQ2",
  "gene_name": "Kinesin-like protein KIF9"
}